{
  "term_label": "peptidyl-prolyl cis-trans isomerase activity",
  "gene_symbol": "PPID",
  "gene": "UniProtKB:Q08752",
  "gene_name": "Peptidyl-prolyl cis-trans isomerase D",
  "term_id": "GO:0003755"
}